{
  "term_label": "Unknown biological process",
  "term_id": "UNKNOWN:0002",
  "gene_symbol": "AHCTF1",
  "gene_name": "Protein ELYS",
  "gene": "UniProtKB:Q8WYP5"
}